negative regulation of nucleotide-binding oligomerization domain containing 1 signaling pathway [GO:0070429] (biological process) Definition: Any process that stops, prevents, or reduces the frequency, rate, or extent of the nucleotide-binding oligomerization domain containing 1 (NOD1) pathway. Sources: GOC:add Also known as: negative regulation of NOD1 signaling pathway, negative regulation of nucleotide-binding oligomerization domain containing 1 signalling pathway Relationships: is a type of negative regulation of nucleotide-binding domain, leucine rich repeat containing receptor signaling pathway [GO:0070425]; is a type of GO:0070428; negatively regulates GO:0070427